{
  "gene_name": "Putative uncharacterized protein CIRBP-AS1",
  "term_id": "UNKNOWN:0003",
  "gene_symbol": "CIRBP-AS1",
  "gene": "UniProtKB:Q8TBR5",
  "term_label": "Unknown cellular component"
}